{
  "term_id": "UNKNOWN:0001",
  "gene_symbol": "TMEM170B",
  "gene_name": "Transmembrane protein 170B",
  "gene": "UniProtKB:Q5T4T1",
  "term_label": "Unknown molecular function"
}